{
  "term_id": "GO:0090554",
  "gene": "UniProtKB:P08183",
  "term_label": "phosphatidylcholine floppase activity",
  "gene_symbol": "ABCB1",
  "gene_name": "ATP-dependent translocase ABCB1"
}